{
  "term_id": "UNKNOWN:0003",
  "term_label": "Unknown cellular component",
  "gene_symbol": "TMEM45B",
  "gene": "UniProtKB:Q96B21",
  "gene_name": "Transmembrane protein 45B"
}